aromatic-amino-acid transaminase activity [GO:0008793] (molecular function) Sources: RHEA:17533 Subtypes: GO:0004838, L-phenylalanine-pyruvate transaminase activity [GO:0047312], L-tyrosine-pyruvate transaminase activity [GO:0080098], L-phenylalanine-2-oxoglutarate transaminase activity [GO:0080130] Also known as: aromatic amino acid aminotransferase activity, aromatic amino acid transferase activity, aromatic aminotransferase activity, aromatic-amino-acid:2-oxoglutarate aminotransferase activity, ArAT Relationships: is a type of transaminase activity [GO:0008483] Definition: Catalysis of the reaction: an L-alpha aromatic amino acid + 2-oxoglutarate = an aromatic oxo acid + L-glutamate.